{
  "gene_symbol": "EFCAB3",
  "gene": "UniProtKB:Q8N7B9",
  "term_label": "Unknown cellular component",
  "gene_name": "EF-hand calcium-binding domain-containing protein 3",
  "term_id": "UNKNOWN:0003"
}